hepaticobiliary system development [GO:0061008] (biological process) Sources: GOC:dph Relationships: is a type of system development [GO:0048731] Definition: The progression of the hepaticobiliary system over time, from its formation to the mature structure. The hepaticobiliary system is responsible for metabolic and catabolic processing of small molecules absorbed from the blood or gut, hormones and serum proteins, detoxification, storage of glycogen, triglycerides, metals and lipid soluble vitamins and excretion of bile. Included are the synthesis of albumin, blood coagulation factors, complement, and specific binding proteins. Also known as: hepatobiliary system development